{
  "term_id": "GO:0005549",
  "gene_name": "Olfactory receptor 5AU1",
  "gene": "UniProtKB:Q8NGC0",
  "term_label": "odorant binding",
  "gene_symbol": "OR5AU1"
}